{
  "term_id": "GO:0006281",
  "gene_name": "General transcription factor IIH subunit 1",
  "gene_symbol": "GTF2H1",
  "gene": "UniProtKB:P32780",
  "term_label": "DNA repair"
}